{
  "gene": "UniProtKB:O75487",
  "term_label": "synapse",
  "gene_name": "Glypican-4",
  "term_id": "GO:0045202",
  "gene_symbol": "GPC4"
}